{
  "gene_name": "Acyl-coenzyme A diphosphatase FITM2",
  "gene_symbol": "FITM2",
  "gene": "UniProtKB:Q8N6M3",
  "term_id": "GO:0034389",
  "term_label": "lipid droplet organization"
}